{
  "gene_symbol": "BYSL",
  "gene": "UniProtKB:Q13895",
  "gene_name": "Bystin",
  "term_id": "GO:0006364",
  "term_label": "rRNA processing"
}